regulation of formin-nucleated actin cable assembly [GO:0090337] (biological process) Relationships: is_a regulation of actin filament bundle assembly [GO:0032231]; regulates GO:0070649 References: PMID:12810699, PMID:15923184 Sources: GOC:jh, GOC:tb Subtypes: GO:0090338, negative regulation of formin-nucleated actin cable assembly [GO:0090339] Definition: Any process that modulates the rate, frequency, or extent of formin-nucleated actin cable assembly. Formin-nucleated actin cable assembly is the aggregation, arrangement and bonding together of a set of components to form a formin-nucleated actin cable. A formin-nucleated actin cable is an actin filament bundle that consists of short filaments organized into bundles of uniform polarity, and is nucleated by formins.